{
  "term_id": "GO:0005737",
  "gene_name": "E3 ubiquitin-protein ligase UBR4",
  "gene": "UniProtKB:Q5T4S7",
  "term_label": "cytoplasm",
  "gene_symbol": "UBR4"
}